myoblast migration [GO:0051451] (biological process) Definition: The orderly movement of a myoblast from one site to another, often during the development of a multicellular organism. A myoblast is a cell type that, by fusion with other myoblasts, gives rise to the myotubes that eventually develop into skeletal muscle fibers. Subtypes: GO:0014839 Relationships: is a type of muscle cell migration [GO:0014812] Sources: CL:0000056, GOC:ai, GOC:mtg_muscle